{
  "gene_name": "Zinc finger protein 136",
  "gene": "UniProtKB:P52737",
  "gene_symbol": "ZNF136",
  "term_label": "DNA-binding transcription factor activity, RNA polymerase II-specific",
  "term_id": "GO:0000981"
}